{
  "term_label": "axon",
  "gene_name": "POTE ankyrin domain family member F",
  "term_id": "GO:0030424",
  "gene": "UniProtKB:A5A3E0",
  "gene_symbol": "POTEF"
}